C21-steroid hormone biosynthetic process [GO:0006700] (biological process) Subtypes: progesterone biosynthetic process [GO:0006701], aldosterone biosynthetic process [GO:0032342] Also known as: C21-steroid hormone anabolism, C21-steroid hormone biosynthesis, C21-steroid hormone formation, C21-steroid hormone synthesis Sources: GOC:ai Relationships: is a type of C21-steroid hormone metabolic process [GO:0008207]; is a type of hormone biosynthetic process [GO:0042446]; is a type of steroid hormone biosynthetic process [GO:0120178] Definition: The chemical reactions and pathways resulting in the formation of C21-steroid hormones, steroid compounds containing 21 carbons which function as hormones.